{
  "gene": "UniProtKB:O15466",
  "gene_name": "Alpha-2,8-sialyltransferase 8E",
  "gene_symbol": "ST8SIA5",
  "term_label": "alpha-N-acetylneuraminate alpha-2,8-sialyltransferase activity",
  "term_id": "GO:0003828"
}